{
  "term_id": "UNKNOWN:0003",
  "gene_name": "T cell receptor alpha joining 44 (Fragment)",
  "gene": "UniProtKB:A0A075B6X8",
  "term_label": "Unknown cellular component",
  "gene_symbol": "TRAJ44"
}